{
  "gene_symbol": "KBTBD4",
  "gene_name": "Kelch repeat and BTB domain-containing protein 4",
  "term_id": "UNKNOWN:0003",
  "gene": "UniProtKB:Q9NVX7",
  "term_label": "Unknown cellular component"
}